{
  "term_label": "RNA polymerase II cis-regulatory region sequence-specific DNA binding",
  "gene_symbol": "BATF2",
  "gene_name": "Basic leucine zipper transcriptional factor ATF-like 2",
  "gene": "UniProtKB:Q8N1L9",
  "term_id": "GO:0000978"
}